{
  "gene_name": "Rho guanine nucleotide exchange factor 12",
  "term_label": "G protein-coupled receptor signaling pathway",
  "term_id": "GO:0007186",
  "gene_symbol": "ARHGEF12",
  "gene": "UniProtKB:Q9NZN5"
}